postsynaptic membrane assembly [GO:0097104] (biological process) Definition: The aggregation, arrangement and bonding together of a set of components to form a postsynaptic membrane, a specialized area of membrane facing the presynaptic membrane on the tip of the nerve ending and separated from it by a minute cleft (the synaptic cleft). References: PMID:21424692 Sources: GOC:BHF, GOC:sjp Also known as: post-synaptic membrane assembly Relationships: is a type of postsynaptic membrane organization [GO:0001941]; is a type of membrane assembly [GO:0071709]; is part of GO:0099068